{
  "term_id": "GO:0012505",
  "gene": "UniProtKB:Q13636",
  "gene_name": "Ras-related protein Rab-31",
  "gene_symbol": "RAB31",
  "term_label": "endomembrane system"
}